polar body extrusion after meiotic divisions [GO:0040038] (biological process) Relationships: is a type of meiotic cytokinesis [GO:0033206]; is part of female meiotic nuclear division [GO:0007143] Definition: The cell cycle process in which two small cells are generated, as byproducts destined to degenerate, as a result of the first and second meiotic divisions of a primary oocyte during its development to a mature ovum. One polar body is formed in the first division of meiosis and the other in the second division; at each division, the cytoplasm divides unequally, so that the polar body is of much smaller size than the developing oocyte. At the second division in which a polar body is formed, the polar body and the developing oocyte each contain a haploid set of chromosomes. Sources: GOC:ems, ISBN:0198506732